{
  "gene_name": "Aldo-keto reductase family 1 member B10",
  "term_label": "aldose reductase (NADPH) activity",
  "gene_symbol": "AKR1B10",
  "term_id": "GO:0004032",
  "gene": "UniProtKB:O60218"
}